{
  "term_id": "GO:0005634",
  "gene_name": "Corepressor interacting with RBPJ 1",
  "term_label": "nucleus",
  "gene": "UniProtKB:Q86X95",
  "gene_symbol": "CIR1"
}